{
  "gene_name": "Pterin-4-alpha-carbinolamine dehydratase",
  "gene": "UniProtKB:P61457",
  "term_id": "GO:0008124",
  "term_label": "4-alpha-hydroxytetrahydrobiopterin dehydratase activity",
  "gene_symbol": "PCBD1"
}